{
  "gene_symbol": "ALG10",
  "gene": "UniProtKB:Q5BKT4",
  "term_id": "GO:0006487",
  "term_label": "protein N-linked glycosylation",
  "gene_name": "Dol-P-Glc:Glc(2)Man(9)GlcNAc(2)-PP-Dol alpha-1,2-glucosyltransferase"
}